{
  "gene_name": "Guanine nucleotide-binding protein subunit beta-4",
  "term_label": "signaling receptor complex adaptor activity",
  "gene": "UniProtKB:Q9HAV0",
  "gene_symbol": "GNB4",
  "term_id": "GO:0030159"
}